skeletal muscle fiber adaptation [GO:0043503] (biological process) Relationships: is a type of cellular response to stimulus [GO:0051716]; is part of skeletal muscle adaptation [GO:0043501] References: PMID:11181628, PMID:11449884, PMID:12605307 Sources: GOC:mtg_muscle Also known as: skeletal muscle fibre plasticity, skeletal myofiber plasticity, skeletal myofibre plasticity, skeletal muscle fiber plasticity Definition: Any process in which the skeletal muscle fibers change their phenotypic profiles in response to altered functional demands and a variety of signals. Muscle fibers are formed by the maturation of myotubes. They can be classed as slow, intermediate/fast or fast.